formaldehyde assimilation via xylulose monophosphate cycle [GO:0019648] (biological process) Also known as: formaldehyde assimilation via xylulose-5-phosphate cycle, formaldehyde fixation cycle Relationships: is a type of GO:0019649; is a type of D-xylulose 5-phosphate metabolic process [GO:0051167] Sources: MetaCyc:P185-PWY Definition: The pathway in which formaldehyde is used as a carbon source in the xylulose monophosphate cycle. Methylotrophic yeasts, but not bacteria, utilize the xylulose monophosphate cycle to fix formaldehyde and convert it into metabolically useful organic compounds.